{
  "gene": "UniProtKB:O95977",
  "gene_name": "Sphingosine 1-phosphate receptor 4",
  "term_id": "GO:0004930",
  "term_label": "G protein-coupled receptor activity",
  "gene_symbol": "S1PR4"
}